{
  "term_id": "UNKNOWN:0001",
  "gene_name": "Uncharacterized protein C20orf141",
  "term_label": "Unknown molecular function",
  "gene": "UniProtKB:Q9NUB4",
  "gene_symbol": "C20orf141"
}